3-methylthiopropyl glucosinolate S-oxygenase activity [GO:0080102] (molecular function) References: PMID:18799661 Relationships: is a type of GO:0016705 Definition: Catalysis of the reaction: 3-methylthiopropyl-glucosinolate = 3-methylsulfinylpropyl-glucosinolate.